RNA trimethylguanosine cap binding [GO:0000341] (molecular function) Definition: Binding to the trimethylguanosine (m(3)(2,2,7)-GTP) group located at the 5' end of some RNA molecules. Such trimethylated cap structures, generally produced by posttranscriptional modification of a 7-methylguanosine cap, are often found on snRNAs and snoRNAs transcribed by RNA polymerase II, but have also be found on snRNAs transcribed by RNA polymerase III. They have also been found on a subset of the mRNA population in some species, e.g. C. elegans. Sources: GOC:krc Also known as: RNA m2,2,7G cap binding Relationships: is a type of RNA cap binding [GO:0000339]